spinal cord interneuron axon guidance [GO:0097377] (biological process) Definition: The process in which the migration of an axon growth cone of a spinal cord interneuron is directed to a specific target site in response to a combination of attractive and repulsive cues. A spinal cord interneuron is a CNS interneuron located in the spinal cord. Subtypes: dorsal spinal cord interneuron axon guidance [GO:0097378] Sources: CL:0005000, GOC:pr Relationships: is a type of interneuron axon guidance [GO:0097376]